oxidoreductase activity [GO:0016491] (molecular function) Subtypes: monooxygenase activity [GO:0004497], oxygen evolving activity [GO:0010242], steroid dehydrogenase activity [GO:0016229], oxidoreductase activity, acting on CH-OH group of donors [GO:0016614], oxidoreductase activity, acting on the CH-CH group of donors [GO:0016627], GO:0016638, oxidoreductase activity, acting on the CH-NH group of donors [GO:0016645], oxidoreductase activity, acting on NAD(P)H [GO:0016651], oxidoreductase activity, acting on other nitrogenous compounds as donors [GO:0016661], oxidoreductase activity, acting on a sulfur group of donors [GO:0016667], oxidoreductase activity, acting on a heme group of donors [GO:0016675], oxidoreductase activity, acting on diphenols and related substances as donors [GO:0016679], oxidoreductase activity, acting on peroxide as acceptor [GO:0016684], oxidoreductase activity, acting on hydrogen as donor [GO:0016695], oxidoreductase activity, acting on single donors with incorporation of molecular oxygen [GO:0016701], GO:0016705, oxidoreductase activity, acting on superoxide radicals as acceptor [GO:0016721], GO:0016722, oxidoreductase activity, acting on CH or CH2 groups [GO:0016725], oxidoreductase activity, acting on iron-sulfur proteins as donors [GO:0016730], oxidoreductase activity, acting on reduced flavodoxin as donor [GO:0016737], oxidoreductase activity, acting on the aldehyde or oxo group of donors [GO:0016903], pyrogallol hydroxytransferase activity [GO:0018706], oxidoreductase activity, acting on phosphorus or arsenic in donors [GO:0030613], selenate reductase activity [GO:0033797], glycyl-radical enzyme activating activity [GO:0043364], GO:0045550, oxidoreductase activity, acting on X-H and Y-H to form an X-Y bond [GO:0046992], GO:0047143, ortho-trichlorophenol reductive dehalogenase activity [GO:0050781], dioxygenase activity [GO:0051213], oxidoreductase activity, reducing C-O-C group as acceptor [GO:0120546], transmembrane monodehydroascorbate reductase activity [GO:0140575] Also known as: redox activity, oxidoreductase activity, acting on other substrates Relationships: is_a catalytic activity [GO:0003824] Sources: EC:1.-.-.- Definition: Catalysis of an oxidation-reduction (redox) reaction, a reversible chemical reaction in which the oxidation state of an atom or atoms within a molecule is altered. One substrate acts as a hydrogen or electron donor and becomes oxidized, while the other acts as hydrogen or electron acceptor and becomes reduced. Regulation: regulated by regulation of oxidoreductase activity [GO:0051341]; positively regulated by GO:0051353; negatively regulated by GO:0051354